regulation of telomere maintenance via telomerase [GO:0032210] (biological process) Relationships: is a type of regulation of telomere maintenance via telomere lengthening [GO:1904356]; is a type of regulation of DNA biosynthetic process [GO:2000278]; regulates GO:0007004 Definition: Any process that modulates the frequency, rate or extent of the addition of telomeric repeats by telomerase. Subtypes: GO:0032211, positive regulation of telomere maintenance via telomerase [GO:0032212] Sources: GOC:mah